blasticidin-S deaminase activity [GO:0047711] (molecular function) Sources: EC:3.5.4.23, MetaCyc:BLASTICIDIN-S-DEAMINASE-RXN Also known as: blasticidin-S aminohydrolase activity Relationships: is a type of GO:0016814; is a type of deaminase activity [GO:0019239] Definition: Catalysis of the reaction: blasticidin S + H2O = deaminohydroxyblasticidin S + NH3.